{
  "gene_symbol": "BAGE2",
  "gene_name": "B melanoma antigen 2",
  "term_id": "UNKNOWN:0002",
  "term_label": "Unknown biological process",
  "gene": "UniProtKB:Q86Y30"
}